ketone biosynthetic process [GO:0042181] (BP) Definition: The chemical reactions and pathways resulting in the formation of ketones, a class of organic compounds that contain the carbonyl group, CO, and in which the carbonyl group is bonded only to carbon atoms. The general formula for a ketone is RCOR, where R and R are alkyl or aryl groups. Sources: GOC:go_curators Also known as: ketone anabolism, ketone biosynthesis, ketone formation, ketone synthesis Relationships: is a type of ketone metabolic process [GO:0042180]; is a type of small molecule biosynthetic process [GO:0044283] Subtypes: progesterone biosynthetic process [GO:0006701], GO:0009234, chalcone biosynthetic process [GO:0009715], pyrroloquinoline quinone biosynthetic process [GO:0018189], GO:0019242, DIF-1 biosynthetic process [GO:0031148], GO:0032342, cortisol biosynthetic process [GO:0034651], GO:0036184, GO:0042371, tetracycline biosynthetic process [GO:0043644], GO:0045151, GO:0045456, (+)-camphor biosynthetic process [GO:0046211], epothilone biosynthetic process [GO:0050814], aurone biosynthetic process [GO:0051551], GO:0061370, brexanolone biosynthetic process [GO:0062174], GO:0106110, GO:0140781, novofumigatonin biosynthetic process [GO:0140782], viridicatumtoxin biosynthetic process [GO:0140872], paxilline biosynthetic process [GO:0140873], paraherquonin biosynthetic process [GO:0140874], andrastin A biosynthetic process [GO:0140876], conidiogenone biosynthetic process [GO:0140879], asperfuranone biosynthetic process [GO:1900554], GO:1900575, GO:1900602, tensidol A biosynthetic process [GO:1900605], tensidol B biosynthetic process [GO:1900608], averantin biosynthetic process [GO:1900763], naphtho-gamma-pyrone biosynthetic process [GO:1900787], shamixanthone biosynthetic process [GO:1900793], cspyrone B1 biosynthetic process [GO:1900802], helvolic acid biosynthetic process [GO:1900812], monodictyphenone biosynthetic process [GO:1900815], tetracenomycin C biosynthetic process [GO:1901106], granaticin biosynthetic process [GO:1901109], funalenone biosynthetic process [GO:1901366], quinone biosynthetic process [GO:1901663], daunorubicin biosynthetic process [GO:1901771], GO:1901777, 1,5-anhydro-D-fructose biosynthetic process [GO:1901803], GO:1901872, neosartoricin biosynthetic process [GO:1902050], 11-oxo-beta-amyrin biosynthetic process [GO:1902383], glycyrrhetinate biosynthetic process [GO:1902386], undecan-2-one biosynthetic process [GO:1902791], androst-4-ene-3,17-dione biosynthetic process [GO:1903449], xanthone-containing compound biosynthetic process [GO:2001307], kojic acid biosynthetic process [GO:2001317] Regulation: regulated by regulation of ketone biosynthetic process [GO:0010566]